{
  "gene": "UniProtKB:Q9NXB0",
  "gene_symbol": "MKS1",
  "term_label": "cilium assembly",
  "term_id": "GO:0060271",
  "gene_name": "Tectonic-like complex member MKS1"
}